{
  "term_id": "GO:0070314",
  "gene_name": "Augurin",
  "term_label": "G1 to G0 transition",
  "gene_symbol": "ECRG4",
  "gene": "UniProtKB:Q9H1Z8"
}